{
  "term_id": "GO:0001725",
  "gene": "UniProtKB:Q53GG5",
  "gene_symbol": "PDLIM3",
  "gene_name": "PDZ and LIM domain protein 3",
  "term_label": "stress fiber"
}